protein transport into plasma membrane raft [GO:0044861] (biological process) Definition: The directed movement of a protein into a plasma membrane raft. Relationships: is a type of protein transport into membrane raft [GO:0032596]; is a type of protein localization to plasma membrane raft [GO:0044860] Sources: GOC:jl